phosphatidylinositol phosphate biosynthetic process [GO:0046854] (biological process) Relationships: is a type of phosphatidylinositol biosynthetic process [GO:0006661] Sources: ISBN:0198506732 Also known as: PIP biosynthesis, PtdInsP biosynthesis, phosphatidylinositol phosphate biosynthesis, phosphatidylinositol phosphate phosphorylation, phosphoinositide phosphorylation, phosphatidylinositol phosphorylation Definition: The chemical reactions and pathways resulting in the formation of phosphatidylinositol phosphate. Subtypes: GO:0036092, GO:1902635, 1-phosphatidyl-1D-myo-inositol 3,5-bisphosphate biosynthetic process [GO:1903102], phosphatidylinositol 5-phosphate biosynthetic process [GO:1904563]